{
  "gene_name": "Adenosine receptor A3",
  "term_label": "G protein-coupled adenosine receptor signaling pathway",
  "gene": "UniProtKB:P0DMS8",
  "term_id": "GO:0001973",
  "gene_symbol": "ADORA3"
}